histone catabolic process [GO:0036205] (biological process) Sources: GOC:krc Relationships: is a type of protein catabolic process [GO:0030163] Definition: The chemical reactions and pathways resulting in the breakdown of a histone protein by individual cells. Note: This term was created even though it describes a process relating to a group of gene products, because histones are highly conserved proteins that are essential components of cellular chromatin in eukaryotic cells. Also known as: histone protein catabolic process